secondary palate development [GO:0062009] (biological process) Relationships: is a type of roof of mouth development [GO:0060021] Definition: The biological process whose specific outcome is the progression of the secondary palate from an initial condition to its mature state. This process begins with the formation of the structure and ends with the mature structure. The secondary palate is the part of the palate formed from the fusion of the two palatine shelves, extensions of the maxillary prominences. References: PMID:28784960